{
  "term_label": "Unknown cellular component",
  "gene_name": "Putative uncharacterized protein PRO1933",
  "gene": "UniProtKB:Q9H354",
  "term_id": "UNKNOWN:0003",
  "gene_symbol": "PRO1933"
}